{
  "gene": "UniProtKB:P52333",
  "term_id": "GO:0004715",
  "gene_symbol": "JAK3",
  "gene_name": "Tyrosine-protein kinase JAK3",
  "term_label": "non-membrane spanning protein tyrosine kinase activity"
}